{
  "term_id": "UNKNOWN:0002",
  "term_label": "Unknown biological process",
  "gene": "UniProtKB:P42166",
  "gene_symbol": "TMPO",
  "gene_name": "Lamina-associated polypeptide 2, isoform alpha"
}